{
  "gene": "UniProtKB:Q4VXU2",
  "term_id": "GO:0003730",
  "gene_symbol": "PABPC1L",
  "term_label": "mRNA 3'-UTR binding",
  "gene_name": "Polyadenylate-binding protein 1-like"
}